{
  "gene_name": "cGMP-dependent 3',5'-cyclic phosphodiesterase",
  "term_id": "GO:0048471",
  "gene_symbol": "PDE2A",
  "gene": "UniProtKB:O00408",
  "term_label": "perinuclear region of cytoplasm"
}